{
  "term_label": "Unknown cellular component",
  "term_id": "UNKNOWN:0003",
  "gene_symbol": "TMEM242",
  "gene_name": "Transmembrane protein 242",
  "gene": "UniProtKB:Q9NWH2"
}